{
  "gene_symbol": "TRMT61B",
  "gene_name": "tRNA (adenine(58)-N(1))-methyltransferase, mitochondrial",
  "gene": "UniProtKB:Q9BVS5",
  "term_id": "GO:0005739",
  "term_label": "mitochondrion"
}